transcription factor TFIIIC2 complex [GO:0034735] (cellular component) Relationships: is a type of RNA polymerase III transcription regulator complex [GO:0090576]; is part of GO:0000127 References: PMID:11433012 Sources: GOC:mah Definition: A transcription factor complex that forms part of the TFIIIC complex, observed in human; composed of five subunits (GTF3C1/hTFIIIC220/TFIIICalpha, GTF3C2/hTFIIIC110/TFIIICbeta, GTF3C3/hTFIIIC102/TFIIICgamma, GTF3C4/hTFIIIC90/TFIIICdelta and GTF3C5/hTFIIIC63/TFIIICepsilon in human) that together recognize the type 2 RNA polymerase III promoter.